{
  "gene": "UniProtKB:Q5SZD4",
  "gene_name": "Glycine N-acyltransferase-like protein 3",
  "gene_symbol": "GLYATL3",
  "term_label": "Unknown cellular component",
  "term_id": "UNKNOWN:0003"
}